dendrite [GO:0030425] (cellular component) Subtypes: dendritic branch [GO:0044307], sensory dendrite [GO:0071683], apical dendrite [GO:0097440], GO:0097441, GO:0097442, GO:0150001, distal dendrite [GO:0150002], GO:1990635 Definition: A neuron projection that has a short, tapering, morphology. Dendrites receive and integrate signals from other neurons or from sensory stimuli, and conduct nerve impulses towards the axon or the cell body. In most neurons, the impulse is conveyed from dendrites to axon via the cell body, but in some types of unipolar neuron, the impulse does not travel via the cell body. Sources: GOC:aruk, GOC:bc, GOC:dos, GOC:mah, GOC:nln Relationships: is a type of neuron projection [GO:0043005]; is part of dendritic tree [GO:0097447]